{
  "term_label": "natural killer cell activation involved in immune response",
  "gene": "UniProtKB:P05013",
  "gene_name": "Interferon alpha-6",
  "term_id": "GO:0002323",
  "gene_symbol": "IFNA6"
}